regulation of lignin biosynthetic process [GO:1901141] (biological process) Relationships: is a type of regulation of secondary metabolite biosynthetic process [GO:1900376]; is a type of regulation of phenylpropanoid metabolic process [GO:2000762]; regulates lignin biosynthetic process [GO:0009809] Subtypes: regulation of syringal lignin biosynthetic process [GO:1901428] Also known as: regulation of lignin anabolism, regulation of lignin biosynthesis, regulation of lignin formation, regulation of lignin synthesis Definition: Any process that modulates the frequency, rate or extent of lignin biosynthetic process. Sources: GOC:TermGenie